{
  "gene_name": "Alpha-protein kinase 1",
  "gene_symbol": "ALPK1",
  "gene": "UniProtKB:Q96QP1",
  "term_label": "innate immune response",
  "term_id": "GO:0045087"
}